{
  "term_id": "UNKNOWN:0002",
  "gene": "UniProtKB:Q58DX5",
  "term_label": "Unknown biological process",
  "gene_name": "Inactive N-acetylated-alpha-linked acidic dipeptidase-like protein 2",
  "gene_symbol": "NAALADL2"
}